{
  "term_id": "GO:0090427",
  "gene_name": "Stimulated by retinoic acid gene 8 protein homolog",
  "gene_symbol": "STRA8",
  "term_label": "activation of meiosis",
  "gene": "UniProtKB:Q7Z7C7"
}